{
  "term_label": "L-tryptophan 2,3-dioxygenase activity",
  "term_id": "GO:0004833",
  "gene_symbol": "IDO2",
  "gene_name": "Indoleamine 2,3-dioxygenase 2",
  "gene": "UniProtKB:Q6ZQW0"
}